{
  "term_label": "Unknown cellular component",
  "gene_name": "WW domain-containing transcription regulator protein 1",
  "term_id": "UNKNOWN:0003",
  "gene_symbol": "WWTR1",
  "gene": "UniProtKB:Q9GZV5"
}